{
  "term_id": "GO:0070378",
  "term_label": "positive regulation of ERK5 cascade",
  "gene_name": "ALK and LTK ligand 2",
  "gene": "UniProtKB:Q6UX46",
  "gene_symbol": "ALKAL2"
}